{
  "gene": "UniProtKB:Q12965",
  "gene_name": "Unconventional myosin-Ie",
  "gene_symbol": "MYO1E",
  "term_id": "GO:0005902",
  "term_label": "microvillus"
}